atrioventricular bundle cell differentiation [GO:0003167] (biological process) Also known as: AV bundle cell differentiation Relationships: is a type of His-Purkinje system cell differentiation [GO:0060932]; is part of bundle of His development [GO:0003166] Definition: The process in which a relatively unspecialized cell acquires the specialized structural and/or functional features of a cell of the atrioventricular bundle. These cells are specialized cardiomyocytes that transmit signals from the AV node to the cardiac Purkinje fibers. Sources: GOC:mtg_heart